2-hydroxy-6-oxohepta-2,4-dienoate hydrolase activity [GO:0018765] (molecular function) Relationships: is a type of hydrolase activity, acting on acid carbon-carbon bonds, in ketonic substances [GO:0016823] Definition: Catalysis of the reaction: (2Z,4E)-2-hydroxy-6-oxohepta-2,4-dienoate + H2O = (2Z)-2-hydroxypenta-2,4-dienoate + acetate + H+. Sources: RHEA:59220